{
  "term_label": "Unknown biological process",
  "gene_name": "Coiled-coil domain-containing protein 60",
  "gene_symbol": "CCDC60",
  "term_id": "UNKNOWN:0002",
  "gene": "UniProtKB:Q8IWA6"
}